{
  "gene_symbol": "OR10A2",
  "gene_name": "Olfactory receptor 10A2",
  "gene": "UniProtKB:Q9H208",
  "term_label": "plasma membrane",
  "term_id": "GO:0005886"
}